{
  "term_label": "nucleus",
  "term_id": "GO:0005634",
  "gene_name": "Putative methyl-CpG-binding domain protein 3-like 5",
  "gene": "UniProtKB:A6NJ08",
  "gene_symbol": "MBD3L5"
}